{
  "term_label": "cytosol",
  "gene_symbol": "RBP7",
  "gene_name": "Retinoid-binding protein 7",
  "gene": "UniProtKB:Q96R05",
  "term_id": "GO:0005829"
}